{
  "term_label": "Unknown biological process",
  "gene_name": "NEDD4-binding protein 2",
  "term_id": "UNKNOWN:0002",
  "gene_symbol": "N4BP2",
  "gene": "UniProtKB:Q86UW6"
}